(25S)-Delta(4)-dafachronate binding [GO:1902051] (molecular function) Relationships: is a type of carboxylic acid binding [GO:0031406]; is a type of steroid hormone binding [GO:1990239] Definition: Binding to (25S)-Delta(4)-dafachronate. References: PMID:16529801 Sources: GOC:TermGenie